{
  "gene_symbol": "MZT1",
  "term_label": "mitotic spindle assembly",
  "gene_name": "Mitotic-spindle organizing protein 1",
  "gene": "UniProtKB:Q08AG7",
  "term_id": "GO:0090307"
}